{
  "gene_name": "Macrophage scavenger receptor types I and II",
  "term_id": "GO:0001540",
  "gene": "UniProtKB:P21757",
  "gene_symbol": "MSR1",
  "term_label": "amyloid-beta binding"
}